{
  "gene": "UniProtKB:Q9H9K5",
  "term_label": "Unknown biological process",
  "term_id": "UNKNOWN:0002",
  "gene_symbol": "ERVMER34-1",
  "gene_name": "Endogenous retroviral envelope protein HEMO"
}